{
  "gene": "UniProtKB:P80162",
  "term_label": "cellular response to lipopolysaccharide",
  "term_id": "GO:0071222",
  "gene_symbol": "CXCL6",
  "gene_name": "C-X-C motif chemokine 6"
}